{
  "gene": "UniProtKB:O43309",
  "gene_name": "Zinc finger and SCAN domain-containing protein 12",
  "gene_symbol": "ZSCAN12",
  "term_id": "UNKNOWN:0003",
  "term_label": "Unknown cellular component"
}